{
  "gene_symbol": "FECH",
  "gene_name": "Ferrochelatase, mitochondrial",
  "term_label": "mitochondrion",
  "term_id": "GO:0005739",
  "gene": "UniProtKB:P22830"
}